regulation of MyD88-independent toll-like receptor signaling pathway [GO:0034127] (biological process) Relationships: is a type of regulation of toll-like receptor signaling pathway [GO:0034121]; regulates GO:0002756 Definition: Any process that modulates the frequency, rate, or extent of MyD88-independent toll-like receptor signaling pathway. References: PMID:16551253, PMID:17328678 Sources: GOC:add Subtypes: negative regulation of MyD88-independent toll-like receptor signaling pathway [GO:0034128], positive regulation of MyD88-independent toll-like receptor signaling pathway [GO:0034129] Also known as: regulation ofMyD88-independent TLR signaling pathway, regulation ofMyD88-independent toll-like receptor signalling pathway